{
  "gene": "UniProtKB:Q8WXC3",
  "gene_name": "Pyrin domain-containing protein 1",
  "term_id": "UNKNOWN:0001",
  "gene_symbol": "PYDC1",
  "term_label": "Unknown molecular function"
}